{
  "term_label": "cell surface receptor signaling pathway",
  "gene_name": "T cell receptor beta variable 16",
  "gene_symbol": "TRBV16",
  "gene": "UniProtKB:A0A087WV62",
  "term_id": "GO:0007166"
}